{
  "term_id": "GO:0002228",
  "term_label": "natural killer cell mediated immunity",
  "gene": "UniProtKB:P26717",
  "gene_symbol": "KLRC2",
  "gene_name": "NKG2-C type II integral membrane protein"
}